{
  "term_id": "GO:0001501",
  "gene_name": "Extracellular tyrosine-protein kinase PKDCC",
  "term_label": "skeletal system development",
  "gene": "UniProtKB:Q504Y2",
  "gene_symbol": "PKDCC"
}